ecdysone catabolic process [GO:0006708] (biological process) Relationships: is a type of ecdysone metabolic process [GO:0008205]; is a type of sterol catabolic process [GO:0016127]; is a type of alcohol catabolic process [GO:0046164]; is a type of GO:0046344 Also known as: ecdysone breakdown, ecdysone catabolism, ecdysone degradation Definition: The chemical reactions and pathways resulting in the breakdown of ecdysone, (22R)-2-beta,3-beta,14,22,25-pentahydroxycholest-7-en-6-one, an ecdysteroid found in insects. Sources: ISBN:0198506732